{
  "term_id": "GO:0005102",
  "gene_name": "Protein-tyrosine kinase 6",
  "gene_symbol": "PTK6",
  "gene": "UniProtKB:Q13882",
  "term_label": "signaling receptor binding"
}